{
  "gene_name": "WD repeat-containing protein 62",
  "term_label": "centriolar satellite",
  "gene": "UniProtKB:O43379",
  "term_id": "GO:0034451",
  "gene_symbol": "WDR62"
}